{
  "gene_symbol": "IGHD",
  "term_id": "GO:0042571",
  "gene_name": "Immunoglobulin heavy constant delta",
  "term_label": "immunoglobulin complex, circulating",
  "gene": "UniProtKB:P01880"
}